{
  "gene_name": "Zinc finger protein 48",
  "gene_symbol": "ZNF48",
  "term_id": "GO:0000976",
  "term_label": "transcription cis-regulatory region binding",
  "gene": "UniProtKB:Q96MX3"
}